formate-tetrahydrofolate ligase activity [GO:0004329] (molecular function) Definition: Catalysis of the reaction: ATP + formate + tetrahydrofolate = ADP + phosphate + 10-formyltetrahydrofolate. Sources: EC:6.3.4.3 Also known as: 10-formyl-THF synthetase activity, 10-formyltetrahydrofolate synthetase activity, formate:tetrahydrofolate ligase (ADP-forming), formyltetrahydrofolate synthetase activity, tetrahydrofolate formylase activity, tetrahydrofolic formylase activity Relationships: is a type of GO:0016879